{
  "gene": "UniProtKB:Q9HAQ2",
  "gene_symbol": "KIF9",
  "gene_name": "Kinesin-like protein KIF9",
  "term_id": "GO:0005874",
  "term_label": "microtubule"
}